hepatocyte growth factor binding [GO:0036458] (molecular function) Relationships: is a type of growth factor binding [GO:0019838] Sources: GOC:curators Definition: Binding to a hepatocyte growth factor. Also known as: HGF binding